axonal growth cone [GO:0044295] (cellular component) Definition: The migrating motile tip of a growing nerve cell axon. Sources: GOC:jl, NIF_Subcellular:sao203987954 Also known as: axon growth cone Relationships: is a type of growth cone [GO:0030426]